{
  "gene_symbol": "PLPP2",
  "gene": "UniProtKB:O43688",
  "term_label": "phosphatidate phosphatase activity",
  "term_id": "GO:0008195",
  "gene_name": "Phospholipid phosphatase 2"
}